Schwann cell differentiation [GO:0014037] (biological process) Definition: The process in which a relatively unspecialized cell acquires the specialized features of a Schwann cell. Schwann cells are found in the peripheral nervous system, where they insulate neurons and axons, and regulate the environment in which neurons function. Regulation: RO_0002211 by regulation of Schwann cell differentiation [GO:0014038]; negatively regulated by negative regulation of Schwann cell differentiation [GO:0014039]; positively regulated by positive regulation of Schwann cell differentiation [GO:0014040] Relationships: is a type of glial cell differentiation [GO:0010001]; is part of peripheral nervous system development [GO:0007422] Sources: GOC:ef